fast endocytic recycling [GO:0032457] (biological process) Definition: The directed movement of membrane-bounded vesicles from peripheral endocytic compartments back to the plasma membrane where they are recycled for further rounds of transport. References: PMID:16473635 Sources: GOC:ecd Also known as: direct endocytic recycling Relationships: is a type of endocytic recycling [GO:0032456]